protein localization to cell wall [GO:0099613] (biological process) Sources: ISBN:0716731363 Relationships: is a type of GO:1990778 Definition: The process of directing proteins towards the cell-wall.